{
  "gene_symbol": "AMBP",
  "term_label": "plasma membrane",
  "gene_name": "Protein AMBP",
  "term_id": "GO:0005886",
  "gene": "UniProtKB:P02760"
}